fibronectin-tissue transglutaminase complex [GO:0071078] (cellular component) Definition: A protein complex that consists of fibronectin bound to tissue transglutaminase, and is involved in cell adhesion. References: PMID:10684262 Also known as: FN-TGM2 complex Relationships: is a type of plasma membrane protein complex [GO:0098797]; is a type of catalytic complex [GO:1902494]